{
  "term_label": "endothelin B receptor binding",
  "gene": "UniProtKB:P20800",
  "gene_symbol": "EDN2",
  "gene_name": "Endothelin-2",
  "term_id": "GO:0031708"
}